{
  "term_id": "GO:0005739",
  "term_label": "mitochondrion",
  "gene": "UniProtKB:Q9NUT2",
  "gene_name": "Mitochondrial potassium channel ATP-binding subunit",
  "gene_symbol": "ABCB8"
}